{
  "gene_name": "Transmembrane protein 25",
  "gene": "UniProtKB:Q86YD3",
  "term_id": "UNKNOWN:0001",
  "term_label": "Unknown molecular function",
  "gene_symbol": "TMEM25"
}